regulation of fungal-type cell wall (1->3)-alpha-glucan biosynthetic process [GO:0070610] (biological process) Definition: Any process that modulates the frequency, rate or extent of the chemical reactions and pathways resulting in the formation of (1->3)-alpha glucans, compounds composed of glucose residues linked by (1->3)-alpha-D-glucosidic bonds, found in fungal-type cell walls, including those of ascospores. Sources: GOC:mah Also known as: regulation of fungal type cell wall 1,3-alpha-glucan biosynthetic process, regulation of fungal-type cell wall 1,3-alpha-glucan anabolism, regulation of fungal-type cell wall 1,3-alpha-glucan biosynthesis, regulation of fungal-type cell wall 1,3-alpha-glucan formation, regulation of fungal-type cell wall 1,3-alpha-glucan synthesis, regulation of fungal-type cell wall alpha-1,3-glucan anabolism, regulation of fungal-type cell wall alpha-1,3-glucan biosynthesis, regulation of fungal-type cell wall alpha-1,3-glucan biosynthetic process, regulation of fungal-type cell wall alpha-1,3-glucan formation, regulation of fungal-type cell wall alpha-1,3-glucan synthesis Relationships: is a type of regulation of fungal-type cell wall biogenesis [GO:0032995]; is a type of regulation of cell wall (1->3)-alpha-glucan biosynthetic process [GO:0070608]; regulates fungal-type cell wall (1->3)-alpha-glucan biosynthetic process [GO:0070600]